{
  "gene_symbol": "MTURN",
  "term_id": "UNKNOWN:0001",
  "term_label": "Unknown molecular function",
  "gene_name": "Maturin",
  "gene": "UniProtKB:Q8N3F0"
}